{
  "term_label": "protein serine/threonine kinase activity",
  "gene_name": "Testis-specific serine_threonine-protein kinase 4",
  "term_id": "GO:0004674",
  "gene": "UniProtKB:Q6SA08",
  "gene_symbol": "TSSK4"
}